{
  "term_id": "GO:0045252",
  "term_label": "oxoglutarate dehydrogenase complex",
  "gene_symbol": "DLD",
  "gene": "UniProtKB:P09622",
  "gene_name": "Dihydrolipoyl dehydrogenase, mitochondrial"
}